{
  "gene_name": "Adenosine deaminase domain-containing protein 1",
  "term_id": "GO:0003725",
  "gene_symbol": "ADAD1",
  "term_label": "double-stranded RNA binding",
  "gene": "UniProtKB:Q96M93"
}